{
  "term_label": "Ras protein signal transduction",
  "gene_name": "Ras-related protein Ral-B",
  "gene_symbol": "RALB",
  "term_id": "GO:0007265",
  "gene": "UniProtKB:P11234"
}